{
  "gene_symbol": "TMPRSS11D",
  "gene_name": "Transmembrane protease serine 11D",
  "term_label": "protein processing",
  "term_id": "GO:0016485",
  "gene": "UniProtKB:O60235"
}